positive regulation of spermidine biosynthetic process [GO:1901307] (biological process) Sources: GOC:TermGenie, GOC:pm Also known as: activation of spermidine anabolism, activation of spermidine biosynthesis, activation of spermidine formation, activation of spermidine synthesis, positive regulation of spermidine anabolism, positive regulation of spermidine biosynthesis, positive regulation of spermidine formation, positive regulation of spermidine synthesis, up regulation of spermidine anabolism, up regulation of spermidine biosynthesis, up regulation of spermidine biosynthetic process, up regulation of spermidine formation, up regulation of spermidine synthesis, up-regulation of spermidine anabolism, up-regulation of spermidine biosynthesis, up-regulation of spermidine biosynthetic process, up-regulation of spermidine formation, up-regulation of spermidine synthesis, upregulation of spermidine anabolism, upregulation of spermidine biosynthesis, upregulation of spermidine biosynthetic process, upregulation of spermidine formation, upregulation of spermidine synthesis, activation of spermidine biosynthetic process Relationships: is_a GO:0009891; is a type of positive regulation of amine metabolic process [GO:0033240]; is a type of regulation of spermidine biosynthetic process [GO:1901304]; positively regulates spermidine biosynthetic process [GO:0008295] Definition: Any process that activates or increases the frequency, rate or extent of spermidine biosynthetic process.